{
  "gene_symbol": "ERCC1",
  "gene": "UniProtKB:P07992",
  "gene_name": "DNA excision repair protein ERCC-1",
  "term_label": "single-stranded DNA binding",
  "term_id": "GO:0003697"
}